{
  "term_id": "GO:0003713",
  "term_label": "transcription coactivator activity",
  "gene_symbol": "CRTC1",
  "gene": "UniProtKB:Q6UUV9",
  "gene_name": "CREB-regulated transcription coactivator 1"
}